{
  "gene_name": "Histone chaperone ASF1A",
  "gene": "UniProtKB:Q9Y294",
  "gene_symbol": "ASF1A",
  "term_label": "chromatin",
  "term_id": "GO:0000785"
}